{
  "gene_symbol": "ABHD13",
  "gene": "UniProtKB:Q7L211",
  "term_id": "GO:0008474",
  "term_label": "palmitoyl-(protein) hydrolase activity",
  "gene_name": "Protein ABHD13"
}